{
  "gene_name": "E3 ubiquitin-protein ligase HERC2",
  "gene": "UniProtKB:O95714",
  "term_id": "GO:0005737",
  "term_label": "cytoplasm",
  "gene_symbol": "HERC2"
}